{
  "term_id": "GO:0005730",
  "gene_name": "E3 ubiquitin-protein ligase Mdm2",
  "gene": "UniProtKB:Q00987",
  "term_label": "nucleolus",
  "gene_symbol": "MDM2"
}